1-phosphatidylinositol-3-kinase regulator activity [GO:0046935] (molecular function) Also known as: 1-phosphatidylinositol 3-kinase regulator activity, phosphatidylinositol 3-kinase, class I, regulator activity Definition: Modulates the activity of the enzyme 1-phosphatidylinositol-3-kinase activity. Note: See also the molecular function term '1-phosphatidylinositol-3-kinase activity ; GO:0016303'. Sources: GOC:ai Relationships: is_a kinase regulator activity [GO:0019207]; regulates 1-phosphatidylinositol-3-kinase activity [GO:0016303]